cellular response to putrescine [GO:1904586] (biological process) References: PMID:20805360 Sources: GOC:TermGenie, GO_REF:0000071 Also known as: cellular response to 1,4-Butanediamine, cellular response to 1,4-Diaminobutane, cellular response to tetramethylenediamine Definition: Any process that results in a change in state or activity of a cell (in terms of movement, secretion, enzyme production, gene expression, etc.) as a result of a putrescine stimulus. Relationships: is a type of cellular response to nitrogen compound [GO:1901699]; is a type of response to putrescine [GO:1904585]